negative regulation of mRNA splicing, via spliceosome [GO:0048025] (biological process) Also known as: negative regulation of pre-mRNA splicing, down regulation of nuclear mRNA splicing, via spliceosome, down-regulation of nuclear mRNA splicing, via spliceosome, downregulation of nuclear mRNA splicing, via spliceosome, negative regulation of nuclear mRNA splicing, via spliceosome, down regulation of nuclear mRNA splicing via U2-type spliceosome, down-regulation of nuclear mRNA splicing via U2-type spliceosome, downregulation of nuclear mRNA splicing via U2-type spliceosome, inhibition of nuclear mRNA splicing via U2-type spliceosome, inhibition of nuclear mRNA splicing, via spliceosome, negative regulation of nuclear mRNA splicing via U2-type spliceosome Definition: Any process that stops, prevents or reduces the rate or extent of mRNA splicing via a spliceosomal mechanism. Relationships: is a type of negative regulation of RNA splicing [GO:0033119]; is a type of GO:0048024; is a type of negative regulation of mRNA processing [GO:0050686]; negatively regulates mRNA splicing, via spliceosome [GO:0000398] Subtypes: negative regulation of mRNA cis splicing, via spliceosome [GO:1905745] Sources: GOC:jid